{
  "term_id": "GO:0017147",
  "gene_symbol": "FZD1",
  "gene_name": "Frizzled-1",
  "gene": "UniProtKB:Q9UP38",
  "term_label": "Wnt-protein binding"
}